{
  "term_label": "G protein-coupled ADP receptor activity",
  "gene": "UniProtKB:P47900",
  "gene_name": "P2Y purinoceptor 1",
  "gene_symbol": "P2RY1",
  "term_id": "GO:0001621"
}